lysine metabolic process [GO:0006553] (biological process) Definition: The chemical reactions and pathways involving lysine, 2,6-diaminohexanoic acid. Sources: GOC:go_curators Relationships: is a type of GO:1901605 Subtypes: GO:0006554, lysine biosynthetic process [GO:0009085] Also known as: lysine metabolism